necroptotic process [GO:0070266] (biological process) References: PMID:18846107, PMID:20823910, PMID:21737330, PMID:21760595, PMID:21876153 Sources: GOC:BHF, GOC:dph, GOC:mah, GOC:mtg_apoptosis, GOC:tb Regulation: regulated by regulation of necroptotic process [GO:0060544]; positively regulated by positive regulation of necroptotic process [GO:0060545]; negatively regulated by negative regulation of necroptotic process [GO:0060546] Also known as: induction of necroptosis, induction of necroptosis by extracellular signals, induction of necroptosis of activated-T cells, programmed necrosis, programmed necrotic cell death, RIPK1-mediated regulated necrosis, TNF-induced necroptosis, necroptosis, PARP-dependent cell death, activation of necroptosis, activation of necroptosis by extracellular signals, activation of necroptosis in response to extracellular signals, activation of necroptosis of activated-T cells, establishment of necroptosis, establishment of necroptosis of activated-T cells, extracellular signal-induced necroptosis, parthanatos Relationships: is a type of programmed necrotic cell death [GO:0097300] Definition: A programmed necrotic cell death process which begins when a cell receives a signal (e.g. a ligand binding to a death receptor or to a Toll-like receptor), and proceeds through a series of biochemical events (signaling pathways), characterized by activation of receptor-interacting serine/threonine-protein kinase 1 and/or 3 (RIPK1/3, also called RIP1/3) and by critical dependence on mixed lineage kinase domain-like (MLKL), and which typically lead to common morphological features of necrotic cell death. The process ends when the cell has died. The process is divided into a signaling phase, and an execution phase, which is triggered by the former. Note: Examples of this are Birc2 and Birc3 (UniProt symbols Q62210 and O08863) in PMID:21052097.